positive regulation of interleukin-1 alpha production [GO:0032730] (biological process) Sources: GOC:mah Definition: Any process that activates or increases the frequency, rate, or extent of interleukin-1 alpha production. Relationships: is a type of GO:0032650; is a type of GO:0032732; RO_0002213 interleukin-1 alpha production [GO:0032610] Also known as: positive regulation of IL-1 alpha production, up regulation of interleukin-1 alpha production, up-regulation of interleukin-1 alpha production, upregulation of interleukin-1 alpha production, activation of interleukin-1 alpha production, positive regulation of interleukin-1 alpha biosynthetic process, positive regulation of interleukin-1 alpha secretion, stimulation of interleukin-1 alpha production